priRNA 3'-end processing [GO:1990431] (biological process) Relationships: is a type of regulatory ncRNA 3'-end processing [GO:0043628] Also known as: priRNA 3' end processing, primal small RNA 3'-end processing Definition: The process of forming the mature 3' end of a priRNA molecule. References: PMID:24095277